{
  "term_label": "transcription coactivator activity",
  "gene_symbol": "NCOA1",
  "term_id": "GO:0003713",
  "gene_name": "Nuclear receptor coactivator 1",
  "gene": "UniProtKB:Q15788"
}